{
  "term_id": "UNKNOWN:0001",
  "gene": "UniProtKB:Q96Q83",
  "gene_name": "Alpha-ketoglutarate-dependent dioxygenase alkB homolog 3",
  "term_label": "Unknown molecular function",
  "gene_symbol": "ALKBH3"
}